{
  "gene": "UniProtKB:P49770",
  "term_label": "translational initiation",
  "term_id": "GO:0006413",
  "gene_symbol": "EIF2B2",
  "gene_name": "Translation initiation factor eIF-2B subunit beta"
}